{
  "gene_name": "Phosphatase and actin regulator 2",
  "term_id": "GO:0030036",
  "gene_symbol": "PHACTR2",
  "gene": "UniProtKB:O75167",
  "term_label": "actin cytoskeleton organization"
}